{
  "term_id": "GO:0033691",
  "term_label": "sialic acid binding",
  "gene_name": "Sialic acid-binding Ig-like lectin 11",
  "gene_symbol": "SIGLEC11",
  "gene": "UniProtKB:Q96RL6"
}